{
  "term_id": "GO:0007268",
  "gene_name": "Voltage-dependent R-type calcium channel subunit alpha-1E",
  "term_label": "chemical synaptic transmission",
  "gene_symbol": "CACNA1E",
  "gene": "UniProtKB:Q15878"
}